{
  "term_label": "paracellular tight junction channel activity",
  "term_id": "GO:0160187",
  "gene_symbol": "CLDN15",
  "gene_name": "Claudin-15",
  "gene": "UniProtKB:P56746"
}